{
  "gene": "UniProtKB:O43347",
  "term_id": "GO:0007417",
  "gene_symbol": "MSI1",
  "gene_name": "RNA-binding protein Musashi homolog 1",
  "term_label": "central nervous system development"
}